{
  "gene_name": "Ceramide synthase 4",
  "term_label": "sphingosine N-acyltransferase activity",
  "gene": "UniProtKB:Q9HA82",
  "term_id": "GO:0050291",
  "gene_symbol": "CERS4"
}